MAML3-RBP-Jkappa-ICN1 complex [GO:0071179] (CC) Also known as: MAML3-RBP-Jkappa-Notch1 complex Relationships: is a type of nuclear protein-containing complex [GO:0140513] References: PMID:12370315 Definition: A protein complex that consists of the intracellular domain of Notch1 (ICN1), the DNA-binding transcription factor RBP-Jkappa, and the transcriptional coactivator Mastermind-like-3 (MAML3); the complex is involved in transcriptional activation in response to Notch-mediated signaling.